positive regulation of T-helper 17 type immune response [GO:2000318] (biological process) Definition: Any process that activates or increases the frequency, rate or extent of T-helper 17 type immune response. Sources: GOC:BHF, GOC:mah Also known as: positive regulation of Th17 immune response Relationships: is a type of positive regulation of adaptive immune response based on somatic recombination of immune receptors built from immunoglobulin superfamily domains [GO:0002824]; is a type of GO:2000316; positively regulates T-helper 17 type immune response [GO:0072538] Subtypes: positive regulation of T-helper 17 cell differentiation [GO:2000321]